{
  "gene_symbol": "STAT5A",
  "gene_name": "Signal transducer and activator of transcription 5A",
  "gene": "UniProtKB:P42229",
  "term_label": "RNA polymerase II transcription regulator complex",
  "term_id": "GO:0090575"
}